venom-mediated perturbation of blood circulation [GO:0140134] (biological process) Also known as: venom-mediated perturbation of cardiovascular system, venom-mediated perturbation of circulatory system process Subtypes: venom-mediated perturbation of hemostasis [GO:0044483], venom-mediated vasoconstriction [GO:0044499], GO:0044551, venom-mediated reduction of heart rate [GO:0044556], venom-mediated suppression of bradykinin-dependent vasodilation [GO:0140163] Relationships: is a type of venom-mediated perturbation of biological process [GO:0035738] Definition: A process in which an organism alters or subverts the circulation of blood in another organism via the action of a venom. References: PMID:31370142